establishment of cell polarity [GO:0030010] (biological process) Subtypes: cellular bud site selection [GO:0000282], establishment of lymphocyte polarity [GO:0001767], establishment of cell polarity involved in ameboidal cell migration [GO:0003365], establishment of cell polarity involved in growth plate cartilage chondrocyte division [GO:0003424], establishment of neuroblast polarity [GO:0045200], establishment of monopolar cell polarity [GO:0061162], establishment of bipolar cell polarity [GO:0061171], establishment of cell polarity regulating cell shape [GO:0071964], establishment of epithelial cell polarity [GO:0090162] Sources: GOC:mah Regulation: regulated by regulation of establishment of cell polarity [GO:2000114] Relationships: is a type of establishment or maintenance of cell polarity [GO:0007163] Also known as: cell polarization, bud site selection/establishment of cell polarity Definition: The specification and formation of anisotropic intracellular organization or cell growth patterns.